symbiont-mediated perturbation of host response to abiotic stimulus [GO:0033635] (biological process) Sources: GOC:pamgo_curators Also known as: modulation by symbiont of host response to abiotic stimulus Definition: A process in which a symbiont alters or subverts the response of its host to an abiotic (non-living) stimulus. The host is defined as the larger of the organisms involved in a symbiotic interaction. Relationships: is a type of symbiont-mediated perturbation of host process [GO:0044003] Subtypes: GO:0033638